sperm mitochondrial sheath assembly [GO:0120317] (biological process) Relationships: is a type of cellular component assembly [GO:0022607]; is part of GO:0120316 Definition: The assembly and organization of the sperm mitochondrial sheath, the tightly packed helical sheath of ATP-producing mitochondria restricted to the midpiece of the sperm flagellum. References: PMID:32791035 Sources: GOC:krc